{
  "gene_symbol": "CHI3L2",
  "gene_name": "Chitinase-3-like protein 2",
  "term_id": "GO:0005576",
  "term_label": "extracellular region",
  "gene": "UniProtKB:Q15782"
}